{
  "term_label": "Unknown molecular function",
  "gene_symbol": "USP39",
  "term_id": "UNKNOWN:0001",
  "gene_name": "U4_U6.U5 tri-snRNP-associated protein 2",
  "gene": "UniProtKB:Q53GS9"
}